{
  "gene": "UniProtKB:A6NHG9",
  "gene_name": "Olfactory receptor 5H14",
  "gene_symbol": "OR5H14",
  "term_id": "GO:0005549",
  "term_label": "odorant binding"
}